branched-chain-amino-acid transaminase activity [GO:0004084] (molecular function) Sources: EC:2.6.1.42 Relationships: is a type of transaminase activity [GO:0008483] Subtypes: GO:0052654, GO:0052655, L-isoleucine-2-oxoglutarate transaminase activity [GO:0052656] Also known as: branched-chain amino acid aminotransferase activity, L-branched chain amino acid aminotransferase activity, branched-chain amino acid-glutamate transaminase activity, branched-chain aminotransferase activity, branched-chain-amino-acid:2-oxoglutarate aminotransferase activity, glutamate-branched-chain amino acid transaminase activity, transaminase B activity Definition: Catalysis of the reaction: a branched-chain amino acid (L-leucine, L-isoleucine and L-valine) + 2-oxoglutarate = L-glutamate + a 2-oxocarboxylate derived from the branched-chain amino acid.